{
  "gene_symbol": "PLPP4",
  "term_label": "phosphatidate phosphatase activity",
  "gene": "UniProtKB:Q5VZY2",
  "term_id": "GO:0008195",
  "gene_name": "Phospholipid phosphatase 4"
}